mycolate outer membrane [GO:0036407] (cellular component) Definition: A mycolic acid-rich cell outer membrane containing a lipid bilayer and long-chain mycolic acids (hydroxylated branched-chain fatty acids) that are covalently linked to the cell wall peptidoglycan via an arabinogalactan network. Found in mycobacteria and related genera (e.g. corynebacteria). Relationships: is a type of cell outer membrane [GO:0009279] References: PMID:18316738, PMID:18567661 Sources: GOC:bf, GOC:das, GOC:md Also known as: MOM, mycobacterial outer membrane, mycomembrane